{
  "gene": "UniProtKB:Q13018",
  "gene_name": "Secretory phospholipase A2 receptor",
  "term_id": "GO:0043235",
  "gene_symbol": "PLA2R1",
  "term_label": "receptor complex"
}